positive regulation of cap-dependent translational initiation [GO:1903676] (biological process) Definition: Any process that activates or increases the frequency, rate or extent of cap-dependent translational initiation. References: PMID:11959995 Sources: GOC:PARL, GOC:TermGenie, GOC:bf, GO_REF:0000058 Also known as: up regulation of cap-dependent translational initiation, up-regulation of cap-dependent translational initiation, upregulation of cap-dependent translational initiation, activation of cap-dependent translational initiation Relationships: is a type of regulation of cap-dependent translational initiation [GO:1903674]; is a type of positive regulation of cytoplasmic translational initiation [GO:1904690]; positively regulates cap-dependent translational initiation [GO:0002191]